{
  "gene_name": "Exosome complex component RRP42",
  "term_id": "GO:0035925",
  "gene_symbol": "EXOSC7",
  "term_label": "mRNA 3'-UTR AU-rich region binding",
  "gene": "UniProtKB:Q15024"
}